small protein activating enzyme binding [GO:0044388] (molecular function) Definition: Binding to a small protein activating enzyme, such as ubiquitin-activating enzyme. Sources: GOC:jl Relationships: is a type of enzyme binding [GO:0019899] Subtypes: ubiquitin activating enzyme binding [GO:0033134]